{
  "term_label": "cytoplasm",
  "gene_name": "DNA dC-dU-editing enzyme APOBEC-3C",
  "term_id": "GO:0005737",
  "gene": "UniProtKB:Q9NRW3",
  "gene_symbol": "APOBEC3C"
}